{
  "term_label": "signal transduction",
  "term_id": "GO:0007165",
  "gene_name": "Olfactory receptor 7C1",
  "gene": "UniProtKB:O76099",
  "gene_symbol": "OR7C1"
}